{
  "gene_symbol": "FITM2",
  "term_id": "GO:0008654",
  "gene_name": "Acyl-coenzyme A diphosphatase FITM2",
  "term_label": "phospholipid biosynthetic process",
  "gene": "UniProtKB:Q8N6M3"
}